{
  "term_id": "GO:0002250",
  "gene": "UniProtKB:P01562",
  "gene_name": "Interferon alpha-1_13",
  "gene_symbol": "IFNA1",
  "term_label": "adaptive immune response"
}